{
  "term_label": "Unknown cellular component",
  "term_id": "UNKNOWN:0003",
  "gene_name": "Olfactory receptor 4K15",
  "gene_symbol": "OR4K15",
  "gene": "UniProtKB:Q8NH41"
}